long-day photoperiodism, flowering [GO:0048574] (biological process) Also known as: long-day photoperiodic control of flowering, long-day photoperiodic control of flowering time, long-day photoperiodic control of inflorescence development, response to long-day, flowering, response to short-night, flowering, short-night photoperiodism, flowering Relationships: is a type of GO:0048571; is a type of photoperiodism, flowering [GO:0048573] Sources: GOC:jid, GOC:pj, ISBN:0582015952, ISBN:0697037754, ISBN:0709408862 Regulation: positively regulated by positive regulation of long-day photoperiodism, flowering [GO:0048578]; negatively regulated by negative regulation of long-day photoperiodism, flowering [GO:0048579]; regulated by regulation of long-day photoperiodism, flowering [GO:0048586] Definition: A change from the vegetative to the reproductive phase as a result of detection of, or exposure to, a period of light that exceeds the critical day length. The critical day length varies between species. Although the term is long-day is used, most species actually respond to the duration of the night, so that the response will occur when a period of darkness falls short of the number of hours defined by 24 minus the critical day length.